{
  "term_label": "histone H4 acetyltransferase activity",
  "gene": "UniProtKB:Q86UY6",
  "term_id": "GO:0010485",
  "gene_name": "N-alpha-acetyltransferase 40",
  "gene_symbol": "NAA40"
}